{
  "gene_symbol": "PIAS4",
  "gene": "UniProtKB:Q8N2W9",
  "term_id": "GO:0016925",
  "gene_name": "E3 SUMO-protein ligase PIAS4",
  "term_label": "protein sumoylation"
}